regulation of DNA strand resection involved in replication fork processing [GO:0110026] (biological process) Definition: Any process that modulates the frequency, rate or extent of DNA strand resection involved in replication fork processing. References: PMID:28475874 Sources: GOC:mah Subtypes: GO:0106253, negative regulation of DNA strand resection involved in replication fork processing [GO:0110027] Relationships: is a type of regulation of DNA metabolic process [GO:0051052]; regulates GO:0110025